{
  "gene": "UniProtKB:Q96IP4",
  "gene_symbol": "TENT5A",
  "term_id": "GO:1990817",
  "gene_name": "Terminal nucleotidyltransferase 5A",
  "term_label": "poly(A) RNA polymerase activity"
}